{
  "gene": "UniProtKB:Q92630",
  "gene_name": "Dual specificity tyrosine-phosphorylation-regulated kinase 2",
  "gene_symbol": "DYRK2",
  "term_label": "protein serine/threonine kinase activity",
  "term_id": "GO:0004674"
}